nucleobase biosynthetic process [GO:0046112] (biological process) Subtypes: GO:0009113, pyrimidine nucleobase biosynthetic process [GO:0019856] Definition: The chemical reactions and pathways resulting in the formation of a nucleobase, a nitrogenous base that is a constituent of a nucleic acid. Sources: GOC:ai Relationships: is a type of GO:0009058; is a type of nucleobase metabolic process [GO:0009112] Also known as: nucleobase anabolism, nucleobase biosynthesis, nucleobase formation, nucleobase synthesis